{
  "gene": "UniProtKB:A0A1B0GTS1",
  "gene_symbol": "HSFX4",
  "gene_name": "Heat shock transcription factor, X-linked member 4",
  "term_id": "GO:0000978",
  "term_label": "RNA polymerase II cis-regulatory region sequence-specific DNA binding"
}